{
  "term_label": "Unknown molecular function",
  "gene_name": "Dysbindin",
  "gene": "UniProtKB:Q96EV8",
  "gene_symbol": "DTNBP1",
  "term_id": "UNKNOWN:0001"
}